{
  "gene": "UniProtKB:P25089",
  "term_label": "complement receptor mediated signaling pathway",
  "term_id": "GO:0002430",
  "gene_symbol": "FPR3",
  "gene_name": "N-formyl peptide receptor 3"
}